gibberellin 20-oxidase activity [GO:0045544] (molecular function) References: PMID:32652020, PMID:7604047 Definition: Catalysis of the reaction: 2 2-oxoglutarate + gibberellin A12 (GA12) + H+ + 3 O2 = 3 CO2 + gibberellin A9 (GA9) + 2 H2O + 2 succinate. This reaction results in the oxidation of C-20 gibberellins to form the corresponding C-19 lactones, via a three-step oxidation at C-20 of the GA skeleton. Also converts GA53 to GA20. GA25 is also formed as a minor product. Relationships: is a type of GO:0016706